{
  "term_label": "Unknown cellular component",
  "gene": "UniProtKB:Q01804",
  "gene_symbol": "OTUD4",
  "term_id": "UNKNOWN:0003",
  "gene_name": "OTU domain-containing protein 4"
}